{
  "gene": "UniProtKB:Q9BV87",
  "term_label": "cyclin-dependent protein kinase holoenzyme complex",
  "gene_symbol": "CNPPD1",
  "term_id": "GO:0000307",
  "gene_name": "Protein CNPPD1"
}